{
  "gene_name": "SPATS2-like protein",
  "term_id": "GO:0005737",
  "gene_symbol": "SPATS2L",
  "term_label": "cytoplasm",
  "gene": "UniProtKB:Q9NUQ6"
}